{
  "gene_symbol": "CEP72",
  "gene_name": "Centrosomal protein of 72 kDa",
  "term_id": "GO:1904779",
  "gene": "UniProtKB:Q9P209",
  "term_label": "regulation of protein localization to centrosome"
}